{
  "gene_name": "Inversin",
  "term_id": "GO:1904108",
  "gene": "UniProtKB:Q9Y283",
  "term_label": "protein localization to ciliary inversin compartment",
  "gene_symbol": "INVS"
}